{
  "gene_name": "Cytosolic acyl coenzyme A thioester hydrolase",
  "term_label": "acyl-CoA metabolic process",
  "gene": "UniProtKB:O00154",
  "gene_symbol": "ACOT7",
  "term_id": "GO:0006637"
}